myofibril [GO:0030016] (cellular component) Subtypes: GO:0097512, skeletal muscle myofibril [GO:0098723] Relationships: is a type of contractile muscle fiber [GO:0043292] Sources: ISBN:0815316194 Definition: The contractile element of skeletal and cardiac muscle; a long, highly organized bundle of actin, myosin, and other proteins that contracts by a sliding filament mechanism.